lumenal side of late endosome membrane [GO:0098551] (cellular component) Relationships: is a type of GO:0098565; BFO_0000050 late endosome membrane [GO:0031902] Definition: The side (leaflet) of the late endosome membrane that faces the lumen. Sources: GOC:lr Also known as: internal leaflet of late endosome membrane, internal side of late endosome membrane